{
  "gene_name": "MMS19 nucleotide excision repair protein homolog",
  "gene_symbol": "MMS19",
  "gene": "UniProtKB:Q96T76",
  "term_label": "MMXD complex",
  "term_id": "GO:0071817"
}